{
  "term_id": "GO:0005886",
  "term_label": "plasma membrane",
  "gene_symbol": "FRMPD2",
  "gene_name": "FERM and PDZ domain-containing protein 2",
  "gene": "UniProtKB:Q68DX3"
}